{
  "gene": "UniProtKB:Q6PFW1",
  "term_label": "inositol phosphate biosynthetic process",
  "gene_symbol": "PPIP5K1",
  "gene_name": "Inositol hexakisphosphate and diphosphoinositol-pentakisphosphate kinase 1",
  "term_id": "GO:0032958"
}